{
  "term_id": "GO:0005634",
  "gene_name": "Dual specificity protein phosphatase 16",
  "gene_symbol": "DUSP16",
  "term_label": "nucleus",
  "gene": "UniProtKB:Q9BY84"
}